{
  "term_label": "Unknown molecular function",
  "term_id": "UNKNOWN:0001",
  "gene_symbol": "TRAV1-1",
  "gene": "UniProtKB:A0A0B4J248",
  "gene_name": "T cell receptor alpha variable 1-1"
}